{
  "gene_name": "Putative UPF0607 protein ENSP00000382826",
  "term_id": "UNKNOWN:0002",
  "gene_symbol": "A8MV72",
  "gene": "UniProtKB:A8MV72",
  "term_label": "Unknown biological process"
}